{
  "gene": "UniProtKB:Q9UNQ2",
  "gene_symbol": "DIMT1",
  "gene_name": "Probable dimethyladenosine transferase",
  "term_label": "rRNA methylation",
  "term_id": "GO:0031167"
}